{
  "gene_name": "Mitochondrial assembly of ribosomal large subunit protein 1",
  "term_label": "mitochondrion",
  "gene": "UniProtKB:Q96EH3",
  "gene_symbol": "MALSU1",
  "term_id": "GO:0005739"
}